constitutive secretory pathway [GO:0045054] (biological process) Regulation: regulated by GO:1903433; negatively regulated by negative regulation of constitutive secretory pathway [GO:1903434]; positively regulated by positive regulation of constitutive secretory pathway [GO:1903435] Relationships: is a type of exocytosis [GO:0006887] Also known as: constitutive exocytosis Definition: A process of exocytosis found in all eukaryotic cells, in which transport vesicles destined for the plasma membrane leave the trans-Golgi network in a steady stream. Upon exocytosis, the membrane proteins and lipids in these vesicles provide new components for the plasma membrane, and the soluble proteins inside the vesicles are released into the extracellular space. Sources: GOC:mah, ISBN:0716731363